regulation of interleukin-25 production [GO:0032669] (biological process) References: PMID:27901018 Sources: GOC:mah Also known as: regulation of IL-25 production, regulation of interleukin-25 biosynthetic process, regulation of interleukin-25 secretion Relationships: is a type of GO:0001817; regulates interleukin-25 production [GO:0032629] Definition: Any process that modulates the frequency, rate, or extent of interleukin-25 production. Subtypes: negative regulation of interleukin-25 production [GO:0032709], GO:0032749